positive regulation of myoblast proliferation [GO:2000288] (BP) Definition: Any process that activates or increases the frequency, rate or extent of myoblast proliferation. Sources: GOC:BHF Relationships: is a type of positive regulation of cell population proliferation [GO:0008284]; is a type of regulation of myoblast proliferation [GO:2000291]; positively regulates myoblast proliferation [GO:0051450] Subtypes: positive regulation of cardiac muscle myoblast proliferation [GO:0110024]